alphaV-beta3 integrin-tissue transglutaminase complex [GO:0071089] (cellular component) References: PMID:10684262 Definition: A protein complex that consists of an alphaV-beta3 integrin complex bound to tissue transglutaminase. Also known as: ITGAV-ITGB3-TGM2 complex Relationships: is a type of plasma membrane protein complex [GO:0098797]; is a type of catalytic complex [GO:1902494]